{
  "term_label": "Unknown molecular function",
  "gene": "UniProtKB:Q9Y5P2",
  "gene_name": "Chondrosarcoma-associated gene 2_3 protein",
  "term_id": "UNKNOWN:0001",
  "gene_symbol": "CSAG3"
}